{
  "term_id": "GO:0061844",
  "gene_symbol": "CCL14",
  "term_label": "antimicrobial humoral immune response mediated by antimicrobial peptide",
  "gene": "UniProtKB:Q16627",
  "gene_name": "C-C motif chemokine 14"
}